host cellular component [GO:0018995] (cellular component) Also known as: host organism Definition: Any cellular component of a host cell. The host is an organism in which another organism, for instance a parasite or symbiont, spends part or all of its life cycle and from which it obtains nourishment and/or protection. Subtypes: host cell part [GO:0033643], host extracellular space [GO:0043655], host cell [GO:0043657] Sources: ISBN:0198506732 Relationships: is a type of GO:0044217